{
  "gene": "UniProtKB:P51148",
  "gene_name": "Ras-related protein Rab-5C",
  "term_id": "GO:0003924",
  "gene_symbol": "RAB5C",
  "term_label": "GTPase activity"
}